{
  "term_label": "polyubiquitin modification-dependent protein binding",
  "gene": "UniProtKB:Q9UHD9",
  "gene_name": "Ubiquilin-2",
  "term_id": "GO:0031593",
  "gene_symbol": "UBQLN2"
}